ATP:coenzyme F420 adenylyltransferase activity [GO:0043910] (molecular function) References: PMID:7957247, PMID:8550473 Sources: GOC:jl, MetaCyc:RXN-9385 Definition: Catalysis of the reaction: ATP + factor gamma-F420-2 + H+ = coenzyme F390-A + diphosphate. Also known as: ATP:coenzyme F420 adenyltransferase activity, coenzyme F390-A synthetase activity Relationships: is a type of adenylyltransferase activity [GO:0070566]